{
  "term_id": "GO:0034587",
  "gene_symbol": "TDRD6",
  "term_label": "piRNA processing",
  "gene": "UniProtKB:O60522",
  "gene_name": "Tudor domain-containing protein 6"
}